{
  "gene_symbol": "FHIT",
  "gene_name": "Bis(5'-adenosyl)-triphosphatase",
  "term_label": "diadenosine triphosphate catabolic process",
  "term_id": "GO:0015964",
  "gene": "UniProtKB:P49789"
}